phosphatidylcholine synthase activity [GO:0050520] (molecular function) Relationships: is a type of phosphotransferase activity, for other substituted phosphate groups [GO:0016780] Definition: Catalysis of the reaction: CDP-diacylglycerol + choline = 1,2-diacyl-sn-glycero-3-phosphocholine + CMP + H+. Also known as: CDP-diacylglycerol:choline O-phosphatidyltransferase activity, CDP-diglyceride-choline O-phosphatidyltransferase activity, CDPdiglyceride-choline O-phosphatidyltransferase activity, PC synthase activity Sources: EC:2.7.8.24, RHEA:14597